{
  "gene_name": "Attractin-like protein 1",
  "term_label": "Notch binding",
  "gene_symbol": "ATRNL1",
  "gene": "UniProtKB:Q5VV63",
  "term_id": "GO:0005112"
}